{
  "gene_name": "Ribonuclease P protein subunit p25-like protein",
  "gene": "UniProtKB:Q8N5L8",
  "term_id": "GO:0001682",
  "gene_symbol": "RPP25L",
  "term_label": "tRNA 5'-leader removal"
}